{
  "gene_symbol": "QSOX2",
  "term_id": "GO:0000139",
  "gene": "UniProtKB:Q6ZRP7",
  "term_label": "Golgi membrane",
  "gene_name": "Sulfhydryl oxidase 2"
}